endo-1,3(4)-beta-glucanase activity [GO:0052861] (molecular function) Definition: Catalysis of the endohydrolysis of (1->3)- or (1->4)-linkages in beta-D-glucans when the glucose residue whose reducing group is involved in the linkage to be hydrolyzed is itself substituted at C-3. Substrates include laminarin, lichenin and cereal D-glucans. Relationships: is a type of GO:0052736 Also known as: 1,3-(1,3)-beta-D-glucan 3-glucanohydrolase activity, glucan endo-1,3-beta-glucanase activity, C-3 substituted reducing group, glucan endo-1,4-beta-glucanase activity, C-3 substituted reducing group, laminaranase activity, laminarinase activity Sources: EC:3.2.1.6